{
  "gene_name": "Gamma-aminobutyric acid receptor subunit gamma-3",
  "gene_symbol": "GABRG3",
  "gene": "UniProtKB:Q99928",
  "term_label": "gamma-aminobutyric acid signaling pathway",
  "term_id": "GO:0007214"
}